ammonium transmembrane transporter complex [GO:0110067] (cellular component) Definition: High affinity ammonium transporter complex that enables the transfer of ammonium from one side of a membrane to the other. Relationships: is a type of transmembrane transporter complex [GO:1902495] References: PMID:17026539, PMID:23463773 Sources: GOC:bhm Also known as: AMT1 complex